amino acid kinase activity [GO:0019202] (molecular function) Definition: Catalysis of the transfer of a phosphate group, usually from ATP, to an amino acid substrate. Relationships: is a type of kinase activity [GO:0016301] Subtypes: arginine kinase activity [GO:0004054], aspartate kinase activity [GO:0004072], GO:0004349, GO:0004413, GO:0043744, hydroxylysine kinase activity [GO:0047992] Sources: GOC:jl